{
  "term_label": "cell surface",
  "gene": "UniProtKB:Q9UKX5",
  "term_id": "GO:0009986",
  "gene_name": "Integrin alpha-11",
  "gene_symbol": "ITGA11"
}